{
  "term_label": "intracellularly calcium-gated chloride channel activity",
  "term_id": "GO:0005229",
  "gene_name": "Anoctamin-2",
  "gene_symbol": "ANO2",
  "gene": "UniProtKB:Q9NQ90"
}